{
  "term_id": "GO:0045087",
  "term_label": "innate immune response",
  "gene_name": "Beta-defensin 106",
  "gene": "UniProtKB:Q8N104",
  "gene_symbol": "DEFB106A"
}